positive regulation of smooth muscle cell apoptotic process [GO:0034393] (biological process) Relationships: is a type of positive regulation of muscle cell apoptotic process [GO:0010661]; is a type of GO:0034391; RO_0002213 smooth muscle cell apoptotic process [GO:0034390] Also known as: positive regulation of SMC apoptosis, up regulation of smooth muscle cell apoptosis, up-regulation of smooth muscle cell apoptosis, upregulation of smooth muscle cell apoptosis, activation of smooth muscle cell apoptosis, positive regulation of smooth muscle cell apoptosis, stimulation of smooth muscle cell apoptosis Subtypes: positive regulation of vascular associated smooth muscle cell apoptotic process [GO:1905461] Sources: GOC:BHF, GOC:mtg_apoptosis, GOC:rl Definition: Any process that activates or increases the frequency, rate, or extent of smooth muscle cell apoptotic process.